{
  "term_label": "Unknown molecular function",
  "gene_symbol": "CEP68",
  "term_id": "UNKNOWN:0001",
  "gene": "UniProtKB:Q76N32",
  "gene_name": "Centrosomal protein of 68 kDa"
}